{
  "term_id": "GO:0090090",
  "gene": "UniProtKB:Q9BZ67",
  "gene_name": "FERM domain-containing protein 8",
  "gene_symbol": "FRMD8",
  "term_label": "negative regulation of canonical Wnt signaling pathway"
}